{
  "term_label": "mitochondrion distribution",
  "gene_name": "Trafficking kinesin-binding protein 1",
  "gene": "UniProtKB:Q9UPV9",
  "gene_symbol": "TRAK1",
  "term_id": "GO:0048311"
}